{
  "gene_name": "BTB_POZ domain-containing adapter for CUL3-mediated RhoA degradation protein 1",
  "term_id": "GO:0004842",
  "gene_symbol": "KCTD13",
  "gene": "UniProtKB:Q8WZ19",
  "term_label": "ubiquitin-protein transferase activity"
}